{
  "gene_name": "Centrosomal protein of 192 kDa",
  "term_label": "protein localization to centrosome",
  "gene": "UniProtKB:Q8TEP8",
  "gene_symbol": "CEP192",
  "term_id": "GO:0071539"
}